microtubule bundle maintenance [GO:0062195] (biological process) Definition: The organization process that preserves a microtubule bundle in a stable functional or structural state. Relationships: is a type of cellular component maintenance [GO:0043954] References: PMID:18061564